{
  "term_label": "MHC class II protein complex",
  "term_id": "GO:0042613",
  "gene_symbol": "HLA-DRB4",
  "gene_name": "HLA class II histocompatibility antigen, DR beta 4 chain",
  "gene": "UniProtKB:P13762"
}